{
  "gene": "UniProtKB:A6NDX4",
  "term_label": "Unknown cellular component",
  "gene_symbol": "A6NDX4",
  "term_id": "UNKNOWN:0003",
  "gene_name": "Putative transmembrane protein ENSP00000320207"
}